{
  "gene_symbol": "ADAMTS7",
  "term_label": "extracellular matrix organization",
  "term_id": "GO:0030198",
  "gene_name": "A disintegrin and metalloproteinase with thrombospondin motifs 7",
  "gene": "UniProtKB:Q9UKP4"
}